{
  "term_label": "non-membrane spanning protein tyrosine kinase activity",
  "term_id": "GO:0004715",
  "gene_name": "Megakaryocyte-associated tyrosine-protein kinase",
  "gene": "UniProtKB:P42679",
  "gene_symbol": "MATK"
}